lipid droplet localization to prospore membrane leading edge [GO:0140043] (biological process) Definition: Any process in which a lipid droplet is transported to, or maintained to the prospore membrane leading edge. Relationships: is_a lipid localization [GO:0010876]; is a type of GO:0051668 References: PMID:28011631 Also known as: adiposome localization to FSM membrane leading edge, adiposome localization to ascospore-type prospore membrane leading edge, lipid body localization to FSM membrane leading edge, lipid body localization to ascospore-type prospore membrane leading edge, lipid particle localization to FSM membrane leading edge, lipid particle localization to ascospore-type prospore membrane leading edge, adiposome localization to forespore membrane leading edge, lipid body localization to forespore membrane leading edge, lipid particle localization to forespore membrane leading edge